{
  "term_id": "UNKNOWN:0002",
  "gene_name": "Papilin",
  "gene_symbol": "PAPLN",
  "term_label": "Unknown biological process",
  "gene": "UniProtKB:O95428"
}